{
  "term_id": "UNKNOWN:0001",
  "gene_name": "Protein EVI2B",
  "gene": "UniProtKB:P34910",
  "gene_symbol": "EVI2B",
  "term_label": "Unknown molecular function"
}